{
  "gene_name": "WW domain binding protein 1-like",
  "term_label": "Unknown molecular function",
  "gene_symbol": "WBP1L",
  "term_id": "UNKNOWN:0001",
  "gene": "UniProtKB:Q9NX94"
}